{
  "term_id": "GO:0046839",
  "term_label": "phospholipid dephosphorylation",
  "gene_name": "Phospholipid phosphatase-related protein type 1",
  "gene": "UniProtKB:Q8TBJ4",
  "gene_symbol": "PLPPR1"
}